{
  "term_id": "UNKNOWN:0003",
  "term_label": "Unknown cellular component",
  "gene_name": "Serine-rich and transmembrane domain-containing 2",
  "gene": "UniProtKB:A0A1B0GWG4",
  "gene_symbol": "SERTM2"
}